{
  "term_label": "regulation of transcription by RNA polymerase II",
  "gene_name": "Zinc finger protein 606",
  "gene": "UniProtKB:Q8WXB4",
  "term_id": "GO:0006357",
  "gene_symbol": "ZNF606"
}